{
  "term_id": "GO:0007165",
  "term_label": "signal transduction",
  "gene_symbol": "TAB1",
  "gene_name": "TGF-beta-activated kinase 1 and MAP3K7-binding protein 1",
  "gene": "UniProtKB:Q15750"
}